{
  "gene_symbol": "NDUFB10",
  "gene": "UniProtKB:O96000",
  "term_id": "UNKNOWN:0002",
  "term_label": "Unknown biological process",
  "gene_name": "NADH dehydrogenase [ubiquinone] 1 beta subcomplex subunit 10"
}